{
  "term_label": "Unknown biological process",
  "gene_name": "Calcyphosin-like protein",
  "gene_symbol": "CAPSL",
  "gene": "UniProtKB:Q8WWF8",
  "term_id": "UNKNOWN:0002"
}